{
  "term_id": "UNKNOWN:0001",
  "gene_symbol": "BTBD16",
  "term_label": "Unknown molecular function",
  "gene": "UniProtKB:Q32M84",
  "gene_name": "BTB_POZ domain-containing protein 16"
}